mRNA N-acetyltransferase activity [GO:0106162] (molecular function) References: PMID:30449621 Sources: GOC:sp, RHEA:58480 Relationships: is a type of GO:0008080 Definition: Catalysis of the reaction: a cytidine in mRNA + acetyl-CoA + ATP + H2O = ADP + an N(4)-acetylcytidine in mRNA + CoA + H+ + phosphate.